{
  "gene_name": "Phosphatidylinositol-binding clathrin assembly protein",
  "term_label": "vesicle budding from membrane",
  "gene": "UniProtKB:Q13492",
  "gene_symbol": "PICALM",
  "term_id": "GO:0006900"
}